{
  "term_id": "GO:0071577",
  "gene_symbol": "SLC39A1",
  "gene_name": "Zinc transporter ZIP1",
  "term_label": "zinc ion transmembrane transport",
  "gene": "UniProtKB:Q9NY26"
}